{
  "gene": "UniProtKB:Q9H165",
  "gene_name": "B-cell lymphoma_leukemia 11A",
  "term_id": "GO:2000171",
  "term_label": "negative regulation of dendrite development",
  "gene_symbol": "BCL11A"
}